{
  "gene_symbol": "ST6GAL1",
  "gene": "UniProtKB:P15907",
  "gene_name": "Beta-galactoside alpha-2,6-sialyltransferase 1",
  "term_id": "GO:0018279",
  "term_label": "protein N-linked glycosylation via asparagine"
}